{
  "gene": "UniProtKB:P01909",
  "term_label": "lysosomal membrane",
  "gene_symbol": "HLA-DQA1",
  "gene_name": "HLA class II histocompatibility antigen, DQ alpha 1 chain",
  "term_id": "GO:0005765"
}